response to tetracycline [GO:1901326] (BP) Definition: Any process that results in a change in state or activity of a cell or an organism (in terms of movement, secretion, enzyme production, gene expression, etc.) as a result of a tetracycline stimulus. Sources: GOC:TermGenie Relationships: is a type of response to alcohol [GO:0097305]; is a type of response to ketone [GO:1901654] Subtypes: cellular response to tetracycline [GO:0072746]